phagosome maturation involved in apoptotic cell clearance [GO:0090386] (biological process) Sources: GOC:kmv, GOC:tb Definition: A process that is carried out at the cellular level which results in the arrangement of constituent parts of a phagosome within a cell and contributes to apoptotic cell clearance. Phagosome maturation begins with endocytosis and formation of the early phagosome and ends with the formation of the hybrid organelle, the phagolysosome. Relationships: is a type of GO:0090382; is part of apoptotic cell clearance [GO:0043277]